mitochondrion inheritance [GO:0000001] (biological process) Relationships: is_a organelle inheritance [GO:0048308]; is a type of mitochondrion distribution [GO:0048311] References: PMID:10873824, PMID:11389764 Sources: GOC:mcc Also known as: mitochondrial inheritance Definition: The distribution of mitochondria, including the mitochondrial genome, into daughter cells after mitosis or meiosis, mediated by interactions between mitochondria and the cytoskeleton.